{
  "term_label": "regulation of transcription by RNA polymerase II",
  "term_id": "GO:0006357",
  "gene_symbol": "TCF7L1",
  "gene_name": "Transcription factor 7-like 1",
  "gene": "UniProtKB:Q9HCS4"
}